{
  "term_label": "Unknown biological process",
  "gene_name": "SH2 domain-containing adapter protein D",
  "gene": "UniProtKB:Q96IW2",
  "term_id": "UNKNOWN:0002",
  "gene_symbol": "SHD"
}